G protein-coupled nucleotide receptor activity [GO:0001608] (molecular function) Definition: Combining with a nucleotide and transmitting the signal across the membrane by activating an associated G-protein; promotes the exchange of GDP for GTP on the alpha subunit of a heterotrimeric G-protein complex. Sources: GOC:bf, GOC:dph, IUPHAR_GPCR:1294 Also known as: G protein coupled nucleotide receptor activity, G-protein coupled nucleotide receptor activity, nucleotide receptor activity, G protein coupled, nucleotide receptor activity, G-protein coupled Relationships: is a type of G protein-coupled receptor activity [GO:0004930]